forebrain neuron fate commitment [GO:0021877] (biological process) Definition: The process in which the developmental fate of a cell becomes restricted such that it will develop into a neuron that resides in the forebrain. Subtypes: commitment of multipotent stem cells to neuronal lineage in forebrain [GO:0021898], commitment of neuronal cell to specific neuron type in forebrain [GO:0021902] Relationships: is a type of neuron fate commitment [GO:0048663]; is part of forebrain neuron differentiation [GO:0021879] References: PMID:16226447 Sources: GOC:cls, GOC:dgh, GOC:dph, GOC:jid, GO_REF:0000021